{
  "term_label": "synapse maturation",
  "gene_symbol": "SYBU",
  "term_id": "GO:0060074",
  "gene": "UniProtKB:Q9NX95",
  "gene_name": "Syntabulin"
}